WICH complex [GO:0090535] (cellular component) Definition: An ISWI complex that contains an ATPase subunit of the ISWI family (specifically SNF2H in mammals, which contain two ISWI homologs) and WSTF (Williams Syndrome Transcription Factor). WICH plays roles in regulation of RNAP I and III transcription and in DNA replication and repair. References: PMID:15284901, PMID:16568949, PMID:21810179 Sources: GOC:krc Relationships: is a type of ISWI-type complex [GO:0031010]